{
  "term_id": "GO:0005886",
  "gene": "UniProtKB:Q9UHC9",
  "term_label": "plasma membrane",
  "gene_symbol": "NPC1L1",
  "gene_name": "NPC1-like intracellular cholesterol transporter 1"
}